{
  "term_id": "GO:0004720",
  "gene": "UniProtKB:Q08397",
  "gene_name": "Lysyl oxidase homolog 1",
  "term_label": "protein-lysine 6-oxidase activity",
  "gene_symbol": "LOXL1"
}